{
  "gene_symbol": "RNF8",
  "gene_name": "E3 ubiquitin-protein ligase RNF8",
  "term_id": "GO:0006511",
  "gene": "UniProtKB:O76064",
  "term_label": "ubiquitin-dependent protein catabolic process"
}